{
  "term_id": "UNKNOWN:0002",
  "gene_symbol": "TMEM256",
  "gene": "UniProtKB:Q8N2U0",
  "gene_name": "Transmembrane protein 256",
  "term_label": "Unknown biological process"
}